{
  "gene": "UniProtKB:O76070",
  "term_label": "chemical synaptic transmission",
  "term_id": "GO:0007268",
  "gene_name": "Gamma-synuclein",
  "gene_symbol": "SNCG"
}